{
  "gene": "UniProtKB:Q9HB29",
  "term_id": "GO:0050727",
  "term_label": "regulation of inflammatory response",
  "gene_symbol": "IL1RL2",
  "gene_name": "Interleukin-1 receptor-like 2"
}